{
  "gene_symbol": "LRPAP1",
  "gene_name": "Alpha-2-macroglobulin receptor-associated protein",
  "term_id": "GO:0005801",
  "term_label": "cis-Golgi network",
  "gene": "UniProtKB:P30533"
}